alphaV-beta3 integrin-CD98 complex [GO:0071137] (cellular component) Definition: A protein complex that consists of an alphaV-beta3 integrin complex bound to the cell surface antigen CD98. Relationships: is a type of plasma membrane protein complex [GO:0098797] Also known as: ITGAV-ITGB3-SLC3A2 complex References: PMID:18032696